{
  "gene_name": "Claudin-22",
  "term_label": "Unknown biological process",
  "gene_symbol": "CLDN22",
  "term_id": "UNKNOWN:0002",
  "gene": "UniProtKB:Q8N7P3"
}